regulation of recycling endosome localization within postsynapse [GO:0099158] (biological process) Relationships: is a type of regulation of intracellular transport [GO:0032386]; is_a GO:1903421; regulates GO:0036466 References: PMID:20098723 Sources: GOC:dos Definition: Any process that modulates the frequency, rate or extent of transport or maintenance of location of a postsynaptic recycling endosome within the postsynapse.